{
  "term_id": "GO:0016064",
  "gene_symbol": "CSF2RB",
  "term_label": "immunoglobulin mediated immune response",
  "gene_name": "Cytokine receptor common subunit beta",
  "gene": "UniProtKB:P32927"
}